{
  "term_id": "GO:0043410",
  "term_label": "positive regulation of MAPK cascade",
  "gene_symbol": "FGF18",
  "gene_name": "Fibroblast growth factor 18",
  "gene": "UniProtKB:O76093"
}